{
  "term_label": "plasma membrane",
  "gene": "UniProtKB:Q8N1N2",
  "gene_name": "Dynactin-associated protein",
  "gene_symbol": "DYNAP",
  "term_id": "GO:0005886"
}